Tea1 cell-end complex [GO:0031500] (CC) References: PMID:15936270 Relationships: is a type of microtubule associated complex [GO:0005875]; is part of polarisome [GO:0000133] Definition: A high molecular weight complex characterized in S. pombe containing the cell-end anchoring protein Tea1. This complex is transported to the cell ends by microtubules and is involved in bipolar growth and the maintennce of normal cell polarity.